recombination nodule [GO:0005713] (cellular component) Definition: An electron dense structure that is associated with meiotic chromosomes. Sources: GOC:elh Relationships: is a type of GO:0110165; is part of condensed nuclear chromosome [GO:0000794] Subtypes: early recombination nodule [GO:0005714], late recombination nodule [GO:0005715]